{
  "gene": "UniProtKB:O95478",
  "term_label": "maturation of 5.8S rRNA",
  "gene_symbol": "NSA2",
  "gene_name": "Ribosome biogenesis protein NSA2 homolog",
  "term_id": "GO:0000460"
}